{
  "gene_symbol": "IGHMBP2",
  "gene": "UniProtKB:P38935",
  "term_id": "GO:0005737",
  "gene_name": "DNA-binding protein SMUBP-2",
  "term_label": "cytoplasm"
}